{
  "gene_name": "Iron-sulfur cluster assembly 1 homolog, mitochondrial",
  "term_id": "GO:0016226",
  "gene": "UniProtKB:Q9BUE6",
  "gene_symbol": "ISCA1",
  "term_label": "iron-sulfur cluster assembly"
}